fatty acid derivative catabolic process [GO:1901569] (biological process) Relationships: is a type of lipid catabolic process [GO:0016042]; is a type of fatty acid derivative metabolic process [GO:1901568] Sources: GOC:TermGenie, GOC:pr Subtypes: fatty-acyl-CoA catabolic process [GO:0036115], ketone body catabolic process [GO:0046952], fatty acid primary amide catabolic process [GO:0062127], icosanoid catabolic process [GO:1901523], fatty alcohol catabolic process [GO:1903174] Definition: The chemical reactions and pathways resulting in the breakdown of fatty acid derivative. Also known as: fatty acid derivative breakdown, fatty acid derivative catabolism, fatty acid derivative degradation